{
  "gene": "UniProtKB:Q9Y3C0",
  "term_id": "GO:0071203",
  "term_label": "WASH complex",
  "gene_symbol": "WASHC3",
  "gene_name": "WASH complex subunit 3"
}